{
  "term_id": "UNKNOWN:0002",
  "gene_name": "Transmembrane protein 235",
  "gene_symbol": "TMEM235",
  "term_label": "Unknown biological process",
  "gene": "UniProtKB:A6NFC5"
}